{
  "gene": "UniProtKB:Q03431",
  "gene_name": "Parathyroid hormone_parathyroid hormone-related peptide receptor",
  "term_id": "GO:0008528",
  "term_label": "G protein-coupled peptide receptor activity",
  "gene_symbol": "PTH1R"
}